proteolysis [GO:0006508] (biological process) Sources: GOC:bf, GOC:mah Subtypes: GO:0016485, GO:0033619, proteolysis involved in protein catabolic process [GO:0051603], self proteolysis [GO:0097264] Regulation: regulated by GO:0030162; negatively regulated by negative regulation of proteolysis [GO:0045861]; RO_0002213 by positive regulation of proteolysis [GO:0045862] Also known as: peptidolysis, ATP-dependent proteolysis Relationships: is a type of protein metabolic process [GO:0019538] Note: This term was intentionally placed under 'protein metabolic process ; GO:0019538' rather than 'protein catabolic process ; GO:0030163' to cover all processes centered on breaking peptide bonds, including those involved in protein processing. Definition: The hydrolysis of proteins into smaller polypeptides and/or amino acids by cleavage of their peptide bonds.